{
  "term_id": "GO:0005886",
  "term_label": "plasma membrane",
  "gene_name": "Vomeronasal type-1 receptor 2",
  "gene_symbol": "VN1R2",
  "gene": "UniProtKB:Q8NFZ6"
}